{
  "term_label": "kinesin complex",
  "gene_name": "Kinesin-like protein KIF21A",
  "term_id": "GO:0005871",
  "gene": "UniProtKB:Q7Z4S6",
  "gene_symbol": "KIF21A"
}